{
  "gene_symbol": "KRTAP20-1",
  "term_label": "Unknown biological process",
  "term_id": "UNKNOWN:0002",
  "gene": "UniProtKB:Q3LI63",
  "gene_name": "Keratin-associated protein 20-1"
}